{
  "term_id": "GO:0001525",
  "gene": "UniProtKB:P08648",
  "gene_symbol": "ITGA5",
  "term_label": "angiogenesis",
  "gene_name": "Integrin alpha-5"
}